{
  "term_label": "Unknown cellular component",
  "gene_symbol": "FAM167A-AS1",
  "term_id": "UNKNOWN:0003",
  "gene": "UniProtKB:Q96KT0",
  "gene_name": "Uncharacterized protein FAM167A-AS1"
}